{
  "gene": "UniProtKB:P25787",
  "term_label": "Unknown molecular function",
  "gene_symbol": "PSMA2",
  "term_id": "UNKNOWN:0001",
  "gene_name": "Proteasome subunit alpha type-2"
}